{
  "gene": "UniProtKB:Q8NDF8",
  "term_id": "GO:1990817",
  "term_label": "poly(A) RNA polymerase activity",
  "gene_symbol": "TENT4B",
  "gene_name": "Terminal nucleotidyltransferase 4B"
}